{
  "gene_symbol": "UROC1",
  "term_id": "GO:0006548",
  "gene": "UniProtKB:Q96N76",
  "gene_name": "Urocanate hydratase",
  "term_label": "L-histidine catabolic process"
}